mevalonate kinase activity [GO:0004496] (molecular function) Definition: Catalysis of the reaction: (R)-mevalonate + ATP = (R)-5-phosphomevalonate + ADP + 2 H+. Sources: EC:2.7.1.36, RHEA:17065 Also known as: ATP:(R)-mevalonate 5-phosphotransferase activity, ATP:mevalonate 5-phosphotransferase activity, MVA kinase activity, mevalonate 5-phosphotransferase activity, mevalonate kinase (phosphorylating), mevalonate phosphokinase activity, mevalonic acid kinase activity, mevalonic kinase activity Relationships: is a type of kinase activity [GO:0016301]; is a type of GO:0016773